GCA codon-amino acid adaptor activity [GO:0033455] (molecular function) Note: Note that in the standard genetic code, GCA codes for alanine. Sources: GOC:mah Relationships: is a type of GO:0030533 Definition: A triplet codon-amino acid adaptor activity that recognizes a GCA codon. Also known as: alanine tRNA